{
  "term_id": "GO:0008021",
  "gene_symbol": "RAB13",
  "gene_name": "Ras-related protein Rab-13",
  "term_label": "synaptic vesicle",
  "gene": "UniProtKB:P51153"
}